{
  "term_id": "GO:0005886",
  "gene_name": "Tyrosine-protein kinase Lyn",
  "gene": "UniProtKB:P07948",
  "term_label": "plasma membrane",
  "gene_symbol": "LYN"
}